base-excision repair, AP site formation via deaminated base removal [GO:0097510] (biological process) Relationships: is_a base-excision repair, AP site formation [GO:0006285]; has part deaminated base DNA N-glycosylase activity [GO:0097506] Definition: A base-excision repair, AP site formation process occurring via excision of a deaminated base. References: PMID:18789404 Sources: GOC:al